{
  "gene": "UniProtKB:Q32M45",
  "gene_symbol": "ANO4",
  "gene_name": "Anoctamin-4",
  "term_id": "GO:0005886",
  "term_label": "plasma membrane"
}